{
  "gene_name": "Putative nuclease HARBI1",
  "term_id": "UNKNOWN:0003",
  "gene": "UniProtKB:Q96MB7",
  "term_label": "Unknown cellular component",
  "gene_symbol": "HARBI1"
}